{
  "gene_symbol": "ATP2C1",
  "gene_name": "Calcium-transporting ATPase type 2C member 1",
  "gene": "UniProtKB:P98194",
  "term_id": "GO:0005388",
  "term_label": "P-type calcium transporter activity"
}